{
  "term_id": "GO:0070545",
  "gene_name": "Pescadillo homolog",
  "term_label": "PeBoW complex",
  "gene_symbol": "PES1",
  "gene": "UniProtKB:O00541"
}